{
  "gene": "UniProtKB:Q5CZA5",
  "gene_name": "Zinc finger protein 805",
  "term_label": "nucleus",
  "gene_symbol": "ZNF805",
  "term_id": "GO:0005634"
}